{
  "gene_symbol": "HLA-DMB",
  "gene_name": "HLA class II histocompatibility antigen, DM beta chain",
  "term_label": "antigen processing and presentation of exogenous peptide antigen via MHC class II",
  "gene": "UniProtKB:P28068",
  "term_id": "GO:0019886"
}